uterus morphogenesis [GO:0061038] (biological process) Definition: The process in which anatomical structures of the uterus are generated and organized. Sources: GOC:BHF, GOC:dph Relationships: is a type of developmental process involved in reproduction [GO:0003006]; is a type of animal organ morphogenesis [GO:0009887]; is part of uterus development [GO:0060065]